negative regulation of protein localization to cell leading edge [GO:1905872] (biological process) Also known as: down regulation of protein localisation in cell leading edge, down regulation of protein localisation to cell leading edge, down regulation of protein localization in cell leading edge, down regulation of protein localization to cell leading edge, down-regulation of protein localisation in cell leading edge, down-regulation of protein localisation to cell leading edge, down-regulation of protein localization in cell leading edge, down-regulation of protein localization to cell leading edge, downregulation of protein localisation in cell leading edge, downregulation of protein localisation to cell leading edge, downregulation of protein localization in cell leading edge, downregulation of protein localization to cell leading edge, negative regulation of protein localisation in cell leading edge, negative regulation of protein localisation to cell leading edge, negative regulation of protein localization in cell leading edge, inhibition of protein localisation in cell leading edge, inhibition of protein localisation to cell leading edge, inhibition of protein localization in cell leading edge, inhibition of protein localization to cell leading edge Definition: Any process that stops, prevents or reduces the frequency, rate or extent of protein localization to cell leading edge. References: PMID:26324884 Sources: GOC:TermGenie, GO_REF:0000058 Relationships: is a type of negative regulation of protein localization [GO:1903828]; is a type of regulation of protein localization to cell leading edge [GO:1905871]; negatively regulates protein localization to cell leading edge [GO:1902463]